positive regulation of cerebral blood circulation [GO:0120277] (biological process) Relationships: is_a GO:0120276; is a type of positive regulation of blood circulation [GO:1903524]; positively regulates cerebral blood circulation [GO:0120275] Definition: Any process that activates or increases the frequency, rate or extent of cerebral blood circulation. References: PMID:25397684 Sources: GOC:krc Also known as: positive regulation of cerebrum blood circulation, positive regulation of telencephalon blood circulation, up regulation of cerebral blood circulation, up-regulation of cerebral blood circulation, upregulation of cerebral blood circulation, activation of cerebral blood circulation